{
  "gene_symbol": "UNC79",
  "gene_name": "Protein unc-79 homolog",
  "term_id": "UNKNOWN:0001",
  "gene": "UniProtKB:Q9P2D8",
  "term_label": "Unknown molecular function"
}